benzene metabolic process [GO:0018910] (biological process) Definition: The chemical reactions and pathways involving benzene, C6H6, a volatile, very inflammable liquid, contained in the naphtha produced by the destructive distillation of coal, from which it is separated by fractional distillation. Sources: GOC:ai Also known as: benzene metabolism Relationships: is a type of GO:0042537; is a type of hydrocarbon metabolic process [GO:0120252] Subtypes: benzene catabolic process [GO:1900996], benzene biosynthetic process [GO:1900997]